{
  "term_id": "UNKNOWN:0003",
  "term_label": "Unknown cellular component",
  "gene_symbol": "FAM74A7",
  "gene": "UniProtKB:A6NL05",
  "gene_name": "Protein FAM74A7"
}